achiasmate meiosis I [GO:0000705] (biological process) Relationships: is a type of GO:0007127 References: PMID:10690419 Sources: GOC:elh, GOC:sart Definition: The first division of meiosis in which homologous chromosomes are paired and segregated from each other, occurring in the constitutive absence of chiasmata. Also known as: achiasmate meiosis I nuclear division